{
  "term_label": "immunoglobulin complex",
  "term_id": "GO:0019814",
  "gene_symbol": "IGKV1-16",
  "gene_name": "Immunoglobulin kappa variable 1-16",
  "gene": "UniProtKB:P04430"
}